{
  "term_label": "plasma membrane",
  "gene_name": "Short transient receptor potential channel 5",
  "gene": "UniProtKB:Q9UL62",
  "term_id": "GO:0005886",
  "gene_symbol": "TRPC5"
}